{
  "term_id": "GO:0006357",
  "gene_symbol": "MLLT6",
  "gene_name": "Protein AF-17",
  "gene": "UniProtKB:P55198",
  "term_label": "regulation of transcription by RNA polymerase II"
}